haptoglobin-hemoglobin complex [GO:0031838] (cellular component) Relationships: is a type of protein-containing complex [GO:0032991] Definition: A protein complex formed by the stable binding of a haptoglobin to hemoglobin. Sources: GOC:mah